nodal binding [GO:0038100] (molecular function) References: PMID:20629020 Sources: GOC:bf Definition: Binding to a nodal protein, a member of the transforming growth factor-beta superfamily. Relationships: is a type of GO:0005515